{
  "term_label": "Golgi apparatus",
  "term_id": "GO:0005794",
  "gene": "UniProtKB:Q14999",
  "gene_name": "Cullin-7",
  "gene_symbol": "CUL7"
}